{
  "gene": "UniProtKB:Q9NPB0",
  "gene_name": "SAYSvFN domain-containing protein 1",
  "gene_symbol": "SAYSD1",
  "term_label": "protein quality control for misfolded or incompletely synthesized proteins",
  "term_id": "GO:0006515"
}